{
  "term_label": "Unknown molecular function",
  "gene_name": "Programmed cell death 1 ligand 1",
  "gene_symbol": "CD274",
  "gene": "UniProtKB:Q9NZQ7",
  "term_id": "UNKNOWN:0001"
}